{
  "gene_name": "Transcription factor SOX-4",
  "term_id": "GO:0000978",
  "term_label": "RNA polymerase II cis-regulatory region sequence-specific DNA binding",
  "gene": "UniProtKB:Q06945",
  "gene_symbol": "SOX4"
}